other organism cell membrane [GO:0044218] (cellular component) Relationships: is a type of other organism part [GO:0044217] Definition: The cell membrane of a secondary organism with which the first organism is interacting. Sources: GOC:jl Also known as: other organism membrane, foreign membrane